{
  "term_id": "GO:0019433",
  "gene_name": "Omega-hydroxyceramide transacylase",
  "gene_symbol": "PNPLA1",
  "gene": "UniProtKB:Q8N8W4",
  "term_label": "triglyceride catabolic process"
}